hydantoin racemase activity [GO:0036348] (molecular function) Relationships: is a type of GO:0016854 Sources: EC:5.1.99.5, InterPro:IPR015942 Definition: Catalysis of the reaction: D-5-monosubstituted hydantoin = L-5-monosubstituted hydantoin.